{
  "gene_name": "Agrin",
  "term_label": "basement membrane",
  "gene_symbol": "AGRN",
  "gene": "UniProtKB:O00468",
  "term_id": "GO:0005604"
}